{
  "gene_name": "Limb region 1 protein homolog",
  "term_id": "GO:0005886",
  "gene": "UniProtKB:Q8WVP7",
  "term_label": "plasma membrane",
  "gene_symbol": "LMBR1"
}